{
  "term_label": "G protein-coupled receptor signaling pathway",
  "term_id": "GO:0007186",
  "gene": "UniProtKB:Q9P1P4",
  "gene_symbol": "TAAR3P",
  "gene_name": "Putative trace amine-associated receptor 3"
}